lymphatic endothelial cell fate commitment [GO:0060838] (biological process) Sources: GOC:dph, GOC:sdb_2009, GOC:tb Definition: The commitment of a venous blood vessel endothelial cell to a lymphatic endothelial cell fate and its capacity to differentiate into a lymphatic endothelial cell. Relationships: is a type of endothelial cell fate commitment [GO:0060839]; BFO_0000050 lymphatic endothelial cell differentiation [GO:0060836]